{
  "gene": "UniProtKB:Q9Y6Q6",
  "gene_symbol": "TNFRSF11A",
  "gene_name": "Tumor necrosis factor receptor superfamily member 11A",
  "term_label": "lymph node development",
  "term_id": "GO:0048535"
}